engulfment of target by autophagosome [GO:0061736] (biological process) Relationships: is a type of membrane invagination [GO:0010324]; is part of autophagosome assembly [GO:0000045] Definition: The membrane invagination process by which an autophagosomal membrane surrounds an object that will be degraded by macroautophagy. Sources: GOC:PARL, GOC:autophagy, GOC:dph, GOC:pad